{
  "term_id": "GO:0001708",
  "gene_symbol": "TBX21",
  "gene": "UniProtKB:Q9UL17",
  "gene_name": "T-box transcription factor TBX21",
  "term_label": "cell fate specification"
}